{
  "gene": "UniProtKB:Q8NGG7",
  "gene_symbol": "OR8A1",
  "term_id": "GO:0007186",
  "term_label": "G protein-coupled receptor signaling pathway",
  "gene_name": "Olfactory receptor 8A1"
}